{
  "gene_symbol": "SEMA7A",
  "gene_name": "Semaphorin-7A",
  "gene": "UniProtKB:O75326",
  "term_id": "GO:0001755",
  "term_label": "neural crest cell migration"
}